ABC-type glutathione S-conjugate transporter activity [GO:0015431] (molecular function) Definition: Catalysis of the reaction: an S-substituted glutathione(in) + ATP + H2O = an S-substituted glutathione(out) + ADP + phosphate + H+. References: PMID:1455517 Sources: RHEA:19121 Also known as: conjugate transporter activity, ATP-dependent glutathione S-conjugate export pump, GS-X pump, MRP1/GS-X pump, glutathione S-conjugate-exporting ATPase activity, ATPase-coupled glutathione S-conjugate transmembrane transporter activity, glutathione S-conjugate-transporting ATPase activity Relationships: is a type of ABC-type transporter activity [GO:0140359]; is a type of sulfur compound transmembrane transporter activity [GO:1901682]